{
  "gene_name": "Keratin-associated protein 12-3",
  "gene": "UniProtKB:P60328",
  "term_id": "UNKNOWN:0002",
  "gene_symbol": "KRTAP12-3",
  "term_label": "Unknown biological process"
}